{
  "term_label": "Unknown molecular function",
  "gene_name": "Solute carrier family 22 member 7",
  "term_id": "UNKNOWN:0001",
  "gene_symbol": "SLC22A7",
  "gene": "UniProtKB:Q9Y694"
}